{
  "gene": "UniProtKB:P04731",
  "gene_symbol": "MT1A",
  "term_label": "cellular response to cadmium ion",
  "term_id": "GO:0071276",
  "gene_name": "Metallothionein-1A"
}